{
  "gene_name": "Exportin-5",
  "term_label": "nucleus",
  "term_id": "GO:0005634",
  "gene_symbol": "XPO5",
  "gene": "UniProtKB:Q9HAV4"
}